regulation of fatty acid beta-oxidation [GO:0031998] (biological process) Definition: Any process that modulates the frequency, rate or extent of fatty acid bbeta-oxidation. Sources: GOC:mah Relationships: is a type of regulation of fatty acid oxidation [GO:0046320]; is a type of regulation of lipid catabolic process [GO:0050994]; regulates fatty acid beta-oxidation [GO:0006635] Subtypes: negative regulation of fatty acid beta-oxidation [GO:0031999], positive regulation of fatty acid beta-oxidation [GO:0032000], GO:1904735